cellular response to glycine [GO:1905430] (biological process) Relationships: is a type of cellular response to amino acid stimulus [GO:0071230]; is a type of GO:1901699; is a type of cellular response to oxygen-containing compound [GO:1901701]; is a type of response to glycine [GO:1905429] References: PMID:18984164 Sources: GOC:TermGenie, GO_REF:0000071 Definition: Any process that results in a change in state or activity of a cell (in terms of movement, secretion, enzyme production, gene expression, etc.) as a result of a glycine stimulus. Also known as: cellular response to Gly, cellular response to aminoacetic acid, cellular response to aminoethanoic acid, cellular response to glycin